{
  "gene": "UniProtKB:P0DOY3",
  "gene_symbol": "IGLC3",
  "term_label": "immunoglobulin mediated immune response",
  "term_id": "GO:0016064",
  "gene_name": "Immunoglobulin lambda constant 3"
}